{
  "term_label": "Unknown cellular component",
  "gene_name": "Beta-1,4-N-acetylgalactosaminyltransferase 3",
  "gene_symbol": "B4GALNT3",
  "term_id": "UNKNOWN:0003",
  "gene": "UniProtKB:Q6L9W6"
}